{
  "gene_symbol": "CDH20",
  "gene": "UniProtKB:Q9HBT6",
  "term_id": "GO:0008013",
  "term_label": "beta-catenin binding",
  "gene_name": "Cadherin-20"
}